proton-transporting two-sector ATPase complex [GO:0016469] (cellular component) Definition: A large protein complex that catalyzes the synthesis or hydrolysis of ATP by a rotational mechanism, coupled to the transport of protons across a membrane. The complex comprises a membrane sector (F0, V0, or A0) that carries out proton transport and a cytoplasmic compartment sector (F1, V1, or A1) that catalyzes ATP synthesis or hydrolysis. Two major types have been characterized: V-type ATPases couple ATP hydrolysis to the transport of protons across a concentration gradient, whereas F-type ATPases, also known as ATP synthases, normally run in the reverse direction to utilize energy from a proton concentration or electrochemical gradient to synthesize ATP. A third type, A-type ATPases have been found in archaea, and are closely related to eukaryotic V-type ATPases but are reversible. References: PMID:16691483 Sources: GOC:mah, ISBN:0716743663 Also known as: hydrogen-transporting two-sector ATPase complex, vacuolar hydrogen-transporting ATPase Relationships: is a type of membrane protein complex [GO:0098796] Subtypes: proton-transporting V-type ATPase complex [GO:0033176], proton-transporting ATP synthase complex [GO:0045259], GO:1990490